{
  "gene_symbol": "TBC1D28",
  "term_id": "UNKNOWN:0003",
  "gene_name": "TBC1 domain family member 28",
  "gene": "UniProtKB:Q2M2D7",
  "term_label": "Unknown cellular component"
}